positive regulation of erythrocyte clearance [GO:0034108] (biological process) Also known as: positive regulation of RBC clearance, positive regulation of red blood cell clearance, positive regulation of neocytolysis References: PMID:12905029, PMID:14754397 Sources: GOC:add Definition: Any process that activates or increases the frequency, rate, or extent of erythrocyte clearance. Relationships: is a type of positive regulation of immune system process [GO:0002684]; is a type of positive regulation of tissue remodeling [GO:0034105]; is a type of regulation of erythrocyte clearance [GO:0034106]; positively regulates erythrocyte clearance [GO:0034102]